{
  "term_label": "nucleus",
  "term_id": "GO:0005634",
  "gene": "UniProtKB:P04150",
  "gene_symbol": "NR3C1",
  "gene_name": "Glucocorticoid receptor"
}